{
  "term_label": "basolateral plasma membrane",
  "term_id": "GO:0016323",
  "gene_symbol": "VSIG1",
  "gene_name": "V-set and immunoglobulin domain-containing protein 1",
  "gene": "UniProtKB:Q86XK7"
}